asparaginyl-tRNAAsn biosynthesis via transamidation [GO:0070680] (BP) Relationships: is a type of GO:0043039 Sources: GOC:mah, MetaCyc:PWY490-4 Definition: A tRNA aminoacylation process in which asparaginyl-tRNAAsn is formed by a tRNA-dependent two-step pathway. In the first step a non-discriminating aspartyl-tRNA synthetase generates the misacylated L-aspartyl-tRNAAsn species, and in the second step it is amidated to the correctly charged L-asparaginyl-tRNAAsn by the heterotrimeric aspartyl-tRNAAsn amidotransferase.